Fanconi anaemia nuclear complex [GO:0043240] (cellular component) References: PMID:12093742 Sources: GOC:jl Also known as: FA complex, FA core complex, FA nuclear complex, Fanconi anaemia complex Definition: A protein complex composed of the Fanconi anaemia (FA) proteins including A, C, E, G and F (FANCA-F). Functions in the activation of the downstream protein FANCD2 by monoubiquitylation, and is essential for protection against chromosome breakage. Relationships: is a type of nuclear protein-containing complex [GO:0140513]